CD20-Lck-Fyn complex [GO:0070331] (cellular component) Definition: A protein complex that contains the cell-surface protein CD20 and the Src family tyrosine kinases Lck and Fyn. Relationships: is a type of intracellular protein-containing complex [GO:0140535]; is a type of GO:1902494 References: PMID:7545683 Sources: GOC:mah